{
  "gene_name": "Adrenocorticotropic hormone receptor",
  "term_label": "cytoplasm",
  "gene": "UniProtKB:Q01718",
  "gene_symbol": "MC2R",
  "term_id": "GO:0005737"
}